{
  "gene_name": "Phosphoribosyl pyrophosphate synthase-associated protein 1",
  "term_id": "GO:0005737",
  "gene": "UniProtKB:Q14558",
  "gene_symbol": "PRPSAP1",
  "term_label": "cytoplasm"
}